{
  "term_id": "UNKNOWN:0001",
  "gene": "UniProtKB:A6ND91",
  "gene_name": "Aspartate dehydrogenase domain-containing protein",
  "gene_symbol": "ASPDH",
  "term_label": "Unknown molecular function"
}